{
  "gene_name": "Homeodomain-interacting protein kinase 1",
  "gene_symbol": "HIPK1",
  "term_id": "GO:0016605",
  "gene": "UniProtKB:Q86Z02",
  "term_label": "PML body"
}